{
  "gene_symbol": "RIPK4",
  "gene": "UniProtKB:P57078",
  "gene_name": "Receptor-interacting serine_threonine-protein kinase 4",
  "term_label": "Unknown molecular function",
  "term_id": "UNKNOWN:0001"
}